regulation of cerebellar granule cell precursor proliferation [GO:0021936] (biological process) References: PMID:15157725 Sources: GOC:cls, GOC:dgh, GOC:dph, GOC:jid, GO_REF:0000021 Relationships: is a type of GO:2000177; regulates cerebellar granule cell precursor proliferation [GO:0021930] Subtypes: positive regulation of cerebellar granule cell precursor proliferation [GO:0021940], GO:0021941 Definition: The process that modulates the frequency, rate or extent of granule cell precursor proliferation.